{
  "term_id": "UNKNOWN:0001",
  "gene_symbol": "SLC25A42",
  "gene": "UniProtKB:Q86VD7",
  "gene_name": "Mitochondrial coenzyme A transporter SLC25A42",
  "term_label": "Unknown molecular function"
}